{
  "gene_symbol": "THAP10",
  "term_label": "Unknown cellular component",
  "gene": "UniProtKB:Q9P2Z0",
  "gene_name": "THAP domain-containing protein 10",
  "term_id": "UNKNOWN:0003"
}